response to L-arginine [GO:1903576] (BP) Definition: Any process that results in a change in state or activity of a cell or an organism (in terms of movement, secretion, enzyme production, gene expression, etc.) as a result of a L-arginine stimulus. References: PMID:6394628 Sources: GOC:TermGenie, GOC:mr, GO_REF:0000071 Relationships: is a type of response to amino acid [GO:0043200]; is a type of response to nitrogen compound [GO:1901698]; is a type of response to oxygen-containing compound [GO:1901700] Subtypes: cellular response to L-arginine [GO:1903577]